positive regulation of cellular response to amino acid starvation [GO:1903833] (biological process) References: PMID:25002487, PMID:7623840 Sources: GOC:TermGenie, GO_REF:0000058 Definition: Any process that activates or increases the frequency, rate or extent of cellular response to amino acid starvation. Relationships: is a type of GO:0032109; is a type of positive regulation of cellular process [GO:0048522]; is a type of GO:1903832; positively regulates cellular response to amino acid starvation [GO:0034198] Also known as: up regulation of cellular response to amino acid starvation, up-regulation of cellular response to amino acid starvation, upregulation of cellular response to amino acid starvation, activation of cellular response to amino acid starvation